{
  "gene": "UniProtKB:A0A6Q8PGS0",
  "gene_symbol": "A0A6Q8PGS0",
  "term_id": "UNKNOWN:0001",
  "term_label": "Unknown molecular function",
  "gene_name": "Uncharacterized protein"
}